{
  "gene_symbol": "SMARCE1",
  "term_id": "GO:0045892",
  "term_label": "negative regulation of DNA-templated transcription",
  "gene_name": "SWI_SNF-related matrix-associated actin-dependent regulator of chromatin subfamily E member 1",
  "gene": "UniProtKB:Q969G3"
}